vascular associated smooth muscle cell differentiation involved in phenotypic switching [GO:1905420] (biological process) References: PMID:25089138 Sources: GOC:BHF, GOC:BHF_miRNA, GOC:TermGenie, GOC:rph, GO_REF:0000060 Also known as: VSMC differentiation involved in phenotypic switching, vascular smooth muscle cell differentiation involved in phenotypic switching, VSMC differentiation involved in phenotypic dimorphism, vascular associated smooth muscle cell differentiation involved in phenotypic dimorphism, vascular smooth muscle cell differentiation involved in phenotypic dimorphism Regulation: RO_0002211 by regulation of vascular associated smooth muscle cell differentiation involved in phenotypic switching [GO:1905930]; negatively regulated by negative regulation of vascular associated smooth muscle cell differentiation involved in phenotypic switching [GO:1905931]; positively regulated by positive regulation of vascular associated smooth muscle cell differentiation involved in phenotypic switching [GO:1905932] Definition: Any vascular smooth muscle cell differentiation that is involved in phenotypic switching. Relationships: is a type of vascular associated smooth muscle cell differentiation [GO:0035886]; is_a GO:0090679